{
  "term_id": "UNKNOWN:0001",
  "term_label": "Unknown molecular function",
  "gene": "UniProtKB:Q9H765",
  "gene_symbol": "ASB8",
  "gene_name": "Ankyrin repeat and SOCS box protein 8"
}